{
  "gene_name": "Heat shock 70 kDa protein 13",
  "gene_symbol": "HSPA13",
  "gene": "UniProtKB:P48723",
  "term_label": "protein folding chaperone",
  "term_id": "GO:0044183"
}